{
  "term_label": "dendrite",
  "gene": "UniProtKB:Q9H3N8",
  "gene_name": "Histamine H4 receptor",
  "term_id": "GO:0030425",
  "gene_symbol": "HRH4"
}